{
  "gene": "UniProtKB:Q9Y3M9",
  "term_label": "DNA-binding transcription factor activity, RNA polymerase II-specific",
  "gene_name": "Zinc finger protein 337",
  "term_id": "GO:0000981",
  "gene_symbol": "ZNF337"
}